{
  "gene_symbol": "PILRA",
  "gene_name": "Paired immunoglobulin-like type 2 receptor alpha",
  "term_label": "Unknown biological process",
  "term_id": "UNKNOWN:0002",
  "gene": "UniProtKB:Q9UKJ1"
}